plastid rRNA transcription [GO:0042794] (biological process) Definition: The synthesis of ribosomal RNA (rRNA) from a plastid DNA template, usually by a specific plastid RNA polymerase. Also known as: rRNA transcription from plastid promoter Relationships: is a type of rRNA transcription [GO:0009303]; is a type of plastid transcription [GO:0042793] Sources: GOC:jl, ISBN:0321000382